{
  "gene_symbol": "CCNDBP1",
  "term_label": "Unknown biological process",
  "gene_name": "Cyclin-D1-binding protein 1",
  "term_id": "UNKNOWN:0002",
  "gene": "UniProtKB:O95273"
}